phospholipid-hydroperoxide glutathione peroxidase activity [GO:0047066] (molecular function) Definition: Catalysis of the reaction: a hydroperoxy polyunsaturated fatty acid + 2 glutathione = a hydroxy polyunsaturated fatty acid + glutathione disulfide + H2O. Relationships: is a type of peroxidase activity [GO:0004601] References: PMID:3978121, PMID:8617728 Sources: RHEA:19057 Also known as: hydroperoxide glutathione peroxidase activity, peroxidation-inhibiting protein activity, phospholipid hydroperoxide glutathione peroxidase activity